response to indolebutyric acid [GO:0080026] (biological process) References: PMID:18725356 Definition: Any process that results in a change in state or activity of a cell or an organism (in terms of movement, secretion, enzyme production, gene expression, etc.) as a result of an indolebutyric acid stimulus. Also known as: response to IBA stimulus, response to indolebutyric acid stimulus, response to indole-3-butyric acid stimulus Subtypes: cellular response to indolebutyric acid stimulus [GO:0071366] Relationships: is a type of GO:0009733; is a type of response to nitrogen compound [GO:1901698]; is a type of GO:1901700